{
  "term_id": "UNKNOWN:0003",
  "gene_symbol": "APEH",
  "gene": "UniProtKB:P13798",
  "term_label": "Unknown cellular component",
  "gene_name": "Acylamino-acid-releasing enzyme"
}